{
  "gene_symbol": "CHRM1",
  "gene": "UniProtKB:P11229",
  "gene_name": "Muscarinic acetylcholine receptor M1",
  "term_id": "GO:0005886",
  "term_label": "plasma membrane"
}